{
  "gene": "UniProtKB:Q8N292",
  "term_label": "B cell proliferation involved in immune response",
  "term_id": "GO:0002322",
  "gene_name": "Protein GAPT",
  "gene_symbol": "GAPT"
}